{
  "gene_name": "COP9 signalosome complex subunit 9",
  "term_label": "Unknown biological process",
  "term_id": "UNKNOWN:0002",
  "gene_symbol": "COPS9",
  "gene": "UniProtKB:Q8WXC6"
}